{
  "term_id": "GO:0045892",
  "gene_symbol": "MAEL",
  "term_label": "negative regulation of DNA-templated transcription",
  "gene_name": "Protein maelstrom homolog",
  "gene": "UniProtKB:Q96JY0"
}